{
  "gene_name": "Neurogenin-1",
  "gene_symbol": "NEUROG1",
  "term_id": "GO:0061564",
  "term_label": "axon development",
  "gene": "UniProtKB:Q92886"
}